{
  "term_id": "UNKNOWN:0001",
  "gene_symbol": "KRTAP8-1",
  "term_label": "Unknown molecular function",
  "gene": "UniProtKB:Q8IUC2",
  "gene_name": "Keratin-associated protein 8-1"
}